{
  "term_id": "GO:0007596",
  "gene_name": "Transmembrane gamma-carboxyglutamic acid protein 1",
  "term_label": "blood coagulation",
  "gene": "UniProtKB:O14668",
  "gene_symbol": "PRRG1"
}